{
  "gene_symbol": "FCER1G",
  "term_id": "GO:0019886",
  "term_label": "antigen processing and presentation of exogenous peptide antigen via MHC class II",
  "gene": "UniProtKB:P30273",
  "gene_name": "High affinity immunoglobulin epsilon receptor subunit gamma"
}